{
  "term_label": "RNA polymerase II transcription regulatory region sequence-specific DNA binding",
  "term_id": "GO:0000977",
  "gene_symbol": "HMX3",
  "gene": "UniProtKB:A6NHT5",
  "gene_name": "Homeobox protein HMX3"
}